NADH dehydrogenase complex (plastoquinone) [GO:0071685] (cellular component) Relationships: is a type of GO:0010598; is a type of NADH dehydrogenase complex [GO:0030964]; is part of GO:0031976 Sources: DOI:10.1078/0176-1617-00593, GOC:mah Definition: An NADH dehydrogenase complex that catalyzes the transfer of electrons to plastoquinone. The complex is involved in the non-photochemical reduction of plastoquinones and the cyclic electron transport around photosystem I, and is found in plastid thylakoids.